negative regulation of macrophage derived foam cell differentiation [GO:0010745] (biological process) Definition: Any process that decreases the rate, frequency or extent of macrophage derived foam cell differentiation. Macrophage derived foam cell differentiation is the process in which a macrophage acquires the specialized features of a foam cell. A foam cell is a type of cell containing lipids in small vacuoles and typically seen in atherosclerotic lesions, as well as other conditions. Sources: GOC:BHF, GOC:add, GOC:dph, GOC:tb Relationships: is a type of regulation of macrophage derived foam cell differentiation [GO:0010743]; is a type of negative regulation of cell differentiation [GO:0045596]; negatively regulates macrophage derived foam cell differentiation [GO:0010742]